{
  "term_label": "diacylglycerol metabolic process",
  "term_id": "GO:0046339",
  "gene_name": "Diacylglycerol kinase beta",
  "gene_symbol": "DGKB",
  "gene": "UniProtKB:Q9Y6T7"
}